{
  "gene_name": "Spermatogenesis-associated protein 31D1",
  "gene_symbol": "SPATA31D1",
  "term_label": "Unknown cellular component",
  "gene": "UniProtKB:Q6ZQQ2",
  "term_id": "UNKNOWN:0003"
}